{
  "gene_name": "T cell receptor alpha variable 1-1",
  "gene_symbol": "TRAV1-1",
  "term_label": "response to bacterium",
  "gene": "UniProtKB:A0A0B4J248",
  "term_id": "GO:0009617"
}